{
  "gene_name": "SPOC domain-containing protein 1",
  "term_id": "GO:0030674",
  "gene": "UniProtKB:Q6ZMY3",
  "gene_symbol": "SPOCD1",
  "term_label": "protein-macromolecule adaptor activity"
}